{
  "gene_symbol": "TMEM234",
  "gene_name": "Transmembrane protein 234",
  "term_label": "Unknown cellular component",
  "term_id": "UNKNOWN:0003",
  "gene": "UniProtKB:Q8WY98"
}